{
  "term_id": "UNKNOWN:0002",
  "gene_name": "SNRPN upstream reading frame protein",
  "term_label": "Unknown biological process",
  "gene_symbol": "SNURF",
  "gene": "UniProtKB:Q9Y675"
}